{
  "gene_name": "Polyadenylate-binding protein 1-like",
  "term_id": "UNKNOWN:0002",
  "term_label": "Unknown biological process",
  "gene": "UniProtKB:Q4VXU2",
  "gene_symbol": "PABPC1L"
}